{
  "term_id": "GO:0000902",
  "gene": "UniProtKB:Q9HBT6",
  "gene_name": "Cadherin-20",
  "term_label": "cell morphogenesis",
  "gene_symbol": "CDH20"
}